immune response in gut-associated lymphoid tissue [GO:0002387] (biological process) Sources: GOC:jal, ISBN:0781735149 Relationships: is a type of GO:0006955 Definition: Immune response taking place in the gut-associated lymphoid tissue (GALT). GALT includes Peyer's patches, appendix, and solitary lymph nodules. Also known as: immune response in GALT Subtypes: immune response in Peyer's patch [GO:0002388], tolerance induction in gut-associated lymphoid tissue [GO:0002394], immune response in nasopharyngeal-associated lymphoid tissue [GO:0002395]